{
  "gene_name": "Arf-GAP with GTPase, ANK repeat and PH domain-containing protein 9",
  "gene": "UniProtKB:Q5VTM2",
  "gene_symbol": "AGAP9",
  "term_label": "Unknown biological process",
  "term_id": "UNKNOWN:0002"
}